{
  "gene_symbol": "ZNF442",
  "term_id": "GO:0005634",
  "gene_name": "Zinc finger protein 442",
  "term_label": "nucleus",
  "gene": "UniProtKB:Q9H7R0"
}